clathrin coat of synaptic vesicle [GO:0030129] (cellular component) Definition: A clathrin coat found on a synaptic vesicle. Sources: GOC:mah Relationships: is a type of clathrin vesicle coat [GO:0030125]; is part of synaptic vesicle membrane [GO:0030672]